{
  "gene_name": "F-actin-capping protein subunit alpha-2",
  "term_label": "actin cytoskeleton organization",
  "gene": "UniProtKB:P47755",
  "gene_symbol": "CAPZA2",
  "term_id": "GO:0030036"
}